holo-citrate lyase synthase activity [GO:0050519] (molecular function) Also known as: 2'-(5''-phosphoribosyl)-3'-dephospho-CoA transferase activity, 2'-(5''-triphosphoribosyl)-3'-dephospho-CoA:apo-citrate lyase activity, 2'-(5''-triphosphoribosyl)-3'-dephospho-CoA:apo-citrate lyase adenylyltransferase activity, CitX, holo-ACP synthase activity Definition: Catalysis of the reaction: apo-citrate lyase + 2'-(5''-triphosphoribosyl)-3'-dephospho-CoA = diphosphate + holo-citrate lyase. Relationships: is a type of nucleotidyltransferase activity [GO:0016779] Sources: EC:2.7.7.61, MetaCyc:2.7.7.61-RXN